{
  "gene_symbol": "PWWP4",
  "term_label": "Unknown molecular function",
  "gene_name": "PWWP domain-containing DNA repair factor 4",
  "gene": "UniProtKB:A0A494C071",
  "term_id": "UNKNOWN:0001"
}